{
  "term_id": "GO:0030865",
  "term_label": "cortical cytoskeleton organization",
  "gene_symbol": "RHOG",
  "gene": "UniProtKB:P84095",
  "gene_name": "Rho-related GTP-binding protein RhoG"
}